cellular response to purvalanol A [GO:0072754] (biological process) Definition: Any process that results in a change in state or activity of a cell (in terms of movement, secretion, enzyme production, gene expression, etc.) as a result of a purvalanol A stimulus. Sources: GOC:mah Relationships: is a type of cellular response to purine-containing compound [GO:0071415]; is a type of GO:1901560; is a type of GO:1901699